{
  "term_label": "centriolar satellite",
  "gene_name": "Centrosomal protein of 290 kDa",
  "term_id": "GO:0034451",
  "gene": "UniProtKB:O15078",
  "gene_symbol": "CEP290"
}